{
  "gene_symbol": "ACAD9",
  "term_label": "acyl-CoA dehydrogenase activity",
  "gene": "UniProtKB:Q9H845",
  "term_id": "GO:0003995",
  "gene_name": "Complex I assembly factor ACAD9, mitochondrial"
}